taxadien-5-alpha-ol O-acetyltransferase activity [GO:0050638] (molecular function) Sources: EC:2.3.1.162, RHEA:22028 Relationships: is a type of GO:0016413 Also known as: taxadien-5a-ol O-acetyltransferase activity, acetyl coenzyme A: taxa-4(20),11(12)-dien-5alpha-ol O-acetyl transferase activity, acetyl coenzyme A:taxa-4(20),11(12)-dien-5-alpha-ol O-acetyl transferase activity, acetyl-CoA:taxa-4(20),11-dien-5alpha-ol O-acetyltransferase activity, taxa-4(20),11(12)-dien-5alpha-ol-O-acetyltransferase activity, taxadien-5alpha-ol O-acetyltransferase activity, taxadienol acetyltransferase activity Definition: Catalysis of the reaction: acetyl-CoA + taxa-4(20),11-dien-5alpha-ol = CoA + taxa-4(20),11-dien-5alpha-yl acetate.